{
  "gene_symbol": "CDH8",
  "term_label": "cell-cell adhesion mediated by cadherin",
  "gene_name": "Cadherin-8",
  "term_id": "GO:0044331",
  "gene": "UniProtKB:P55286"
}